{
  "gene_name": "Beta-nerve growth factor",
  "gene_symbol": "NGF",
  "term_id": "GO:0048812",
  "gene": "UniProtKB:P01138",
  "term_label": "neuron projection morphogenesis"
}